{
  "gene_name": "Ubiquitin domain-containing protein TINCR",
  "term_id": "UNKNOWN:0001",
  "gene_symbol": "TINCR",
  "term_label": "Unknown molecular function",
  "gene": "UniProtKB:A0A2R8Y7D0"
}